meiotic spindle checkpoint signaling [GO:0044779] (biological process) Subtypes: meiotic spindle assembly checkpoint signaling [GO:0033316] Definition: A signal transduction process that contributes to a cell cycle checkpoint that delays the metaphase/anaphase transition of a meiotic nuclear division until the spindle is correctly assembled and that the chromosomes are attached to the spindle. Sources: GOC:mtg_cell_cycle Relationships: is a type of spindle checkpoint signaling [GO:0031577]; is a type of meiotic cell cycle checkpoint signaling [GO:0033313]; is a type of negative regulation of metaphase/anaphase transition of meiotic cell cycle [GO:1902103] Also known as: intracellular signal transduction involved in meiotic spindle checkpoint, intracellular signal transduction pathway involved in meiotic spindle checkpoint, intracellular signaling cascade involved in meiotic spindle checkpoint, intracellular signaling pathway involved in meiotic spindle checkpoint, meiotic spindle checkpoint